{
  "term_id": "GO:0005737",
  "gene_symbol": "NACA",
  "term_label": "cytoplasm",
  "gene_name": "Nascent polypeptide-associated complex subunit alpha, muscle-specific form",
  "gene": "UniProtKB:E9PAV3"
}